articular cartilage development [GO:0061975] (biological process) Relationships: is a type of cartilage development [GO:0051216] References: PMID:20097540, PMID:20679519 Also known as: articular cartilage of joint development Definition: The process whose specific outcome is the progression of articular cartilage over time, from its formation to the mature structure. Subtypes: temporomandibular joint articular cartilage development [GO:0061976], GO:0061977